{
  "gene_name": "Putative uncharacterized protein C10orf126",
  "gene_symbol": "C10orf126",
  "term_label": "Unknown molecular function",
  "term_id": "UNKNOWN:0001",
  "gene": "UniProtKB:Q8N4M7"
}